{
  "term_id": "GO:0045944",
  "gene_name": "Putative homeobox protein Meis3-like 2",
  "gene_symbol": "MEIS3P2",
  "term_label": "positive regulation of transcription by RNA polymerase II",
  "gene": "UniProtKB:A8K0S8"
}